{
  "term_id": "GO:0016192",
  "gene_name": "Synaptotagmin-8",
  "gene": "UniProtKB:Q8NBV8",
  "gene_symbol": "SYT8",
  "term_label": "vesicle-mediated transport"
}